{
  "term_id": "GO:1902554",
  "gene_symbol": "STRADB",
  "gene_name": "STE20-related kinase adapter protein beta",
  "term_label": "serine/threonine protein kinase complex",
  "gene": "UniProtKB:Q9C0K7"
}